{
  "gene_name": "Cullin-4B",
  "term_id": "GO:0031625",
  "term_label": "ubiquitin protein ligase binding",
  "gene_symbol": "CUL4B",
  "gene": "UniProtKB:Q13620"
}